regulation of insulin secretion involved in cellular response to glucose stimulus [GO:0061178] (biological process) Also known as: regulation of insulin secretion in response to glucose Relationships: is a type of regulation of insulin secretion [GO:0050796]; is a type of regulation of cellular localization [GO:0060341]; RO_0002211 insulin secretion involved in cellular response to glucose stimulus [GO:0035773] Subtypes: GO:0035774, GO:0061179 Sources: GOC:BHF, GOC:dph Definition: Any process that modulates the frequency, rate or extent of the regulated release of insulin that contributes to the response of a cell to glucose.